{
  "term_label": "mitotic spindle midzone assembly",
  "gene": "UniProtKB:Q9P2G4",
  "gene_symbol": "MAP10",
  "gene_name": "Microtubule-associated protein 10",
  "term_id": "GO:0051256"
}